{
  "gene_symbol": "FAM221A",
  "term_id": "UNKNOWN:0003",
  "gene_name": "Protein FAM221A",
  "gene": "UniProtKB:A4D161",
  "term_label": "Unknown cellular component"
}